{
  "term_label": "Golgi apparatus",
  "term_id": "GO:0005794",
  "gene_name": "ELMO domain-containing protein 1",
  "gene_symbol": "ELMOD1",
  "gene": "UniProtKB:Q8N336"
}